heparan sulfate sulfotransferase activity [GO:0034483] (molecular function) Sources: GOC:mah Relationships: is a type of GO:0050698 Subtypes: heparan sulfate 2-sulfotransferase activity [GO:0004394], [heparan sulfate]-glucosamine 3-sulfotransferase activity [GO:0008467], heparan sulfate N-sulfotransferase activity [GO:0015016], heparan sulfate 6-sulfotransferase activity [GO:0017095] Definition: Catalysis of the reaction: 3'-phosphoadenosine 5'-phosphosulfate + heparan sulfate = adenosine 3',5'-bisphosphate + sulfated heparan sulfate.